{
  "term_id": "GO:0000902",
  "gene": "UniProtKB:Q9Y6N8",
  "term_label": "cell morphogenesis",
  "gene_symbol": "CDH10",
  "gene_name": "Cadherin-10"
}